vistamycin biosynthetic process [GO:1901152] (biological process) Also known as: ribostamycin anabolism, ribostamycin biosynthesis, ribostamycin biosynthetic process, ribostamycin formation, ribostamycin synthesis, vistamycin anabolism, vistamycin biosynthesis, vistamycin formation, vistamycin synthesis Relationships: is a type of aminoglycoside antibiotic biosynthetic process [GO:0030648]; is a type of GO:0046173 Sources: GOC:TermGenie, GOC:yaf, UniPathway:UPA00972 Definition: The chemical reactions and pathways resulting in the formation of vistamycin.